{
  "gene_symbol": "GML",
  "term_id": "UNKNOWN:0002",
  "gene": "UniProtKB:Q99445",
  "gene_name": "Glycosyl-phosphatidylinositol-anchored molecule-like protein",
  "term_label": "Unknown biological process"
}